{
  "gene_name": "Large ribosomal subunit protein uL14",
  "term_label": "cytosolic large ribosomal subunit",
  "gene_symbol": "RPL23",
  "term_id": "GO:0022625",
  "gene": "UniProtKB:P62829"
}